{
  "term_id": "UNKNOWN:0001",
  "gene": "UniProtKB:P35325",
  "term_label": "Unknown molecular function",
  "gene_symbol": "SPRR2B",
  "gene_name": "Small proline-rich protein 2B"
}